{
  "gene": "UniProtKB:O15217",
  "term_id": "UNKNOWN:0003",
  "gene_name": "Glutathione S-transferase A4",
  "gene_symbol": "GSTA4",
  "term_label": "Unknown cellular component"
}